{
  "gene_name": "Zinc finger and BTB domain-containing protein 21",
  "gene_symbol": "ZBTB21",
  "gene": "UniProtKB:Q9ULJ3",
  "term_label": "DNA-binding transcription factor activity, RNA polymerase II-specific",
  "term_id": "GO:0000981"
}